serpin family protein binding [GO:0097655] (molecular function) Definition: Binding to a member of the serpin protein family (serine protease inhibitors or classified inhibitor family I4). Serpins are a broadly distributed family of protease inhibitors that use a conformational change to inhibit target enzymes. They are central in controlling many important proteolytic cascades. The majority of serpins inhibit serine proteases, but serpins that inhibit caspases and papain-like cysteine proteases have also been identified. Rarely, serpins perform a non-inhibitory function; for example, several human serpins function as hormone transporters and certain serpins function as molecular chaperones or tumor suppressors. References: PMID:16737556 Sources: GOC:mr, InterPro:IPR000215 Relationships: is a type of protein binding [GO:0005515]